CGA codon-amino acid adaptor activity [GO:0033431] (molecular function) Relationships: is a type of triplet codon-amino acid adaptor activity [GO:0030533] Also known as: arginine tRNA Definition: A triplet codon-amino acid adaptor activity that recognizes a CGA codon. Note: Note that in the standard genetic code, CGA codes for arginine. Sources: GOC:mah